snRNA export from nucleus [GO:0006408] (biological process) Sources: GOC:ma Definition: The directed movement of snRNA from the nucleus to the cytoplasm. Also known as: snRNA export from cell nucleus, snRNA export out of nucleus, snRNA transport from nucleus to cytoplasm, snRNA-nucleus export Relationships: is a type of RNA export from nucleus [GO:0006405]; is_a snRNA transport [GO:0051030]